{
  "term_label": "lens fiber cell development",
  "gene": "UniProtKB:Q12934",
  "gene_symbol": "BFSP1",
  "gene_name": "Filensin",
  "term_id": "GO:0070307"
}